{
  "gene_symbol": "CLCA1",
  "gene": "UniProtKB:A8K7I4",
  "term_id": "GO:0005886",
  "term_label": "plasma membrane",
  "gene_name": "Calcium-activated chloride channel regulator 1"
}